centripetally migrating follicle cell migration [GO:0060269] (biological process) Relationships: is a type of follicle cell of egg chamber migration [GO:0007297] Definition: The cell migration process in which a follicle cell migrates as part of an epithelial sheet between the nurse cells and the oocyte. At the end of migration, they cover the anterior of the oocyte. Sources: GOC:dph